{
  "gene_name": "Zinc finger protein 366",
  "term_label": "RNA polymerase II cis-regulatory region sequence-specific DNA binding",
  "gene": "UniProtKB:Q8N895",
  "term_id": "GO:0000978",
  "gene_symbol": "ZNF366"
}